{
  "term_id": "GO:1901907",
  "gene_name": "Diphosphoinositol polyphosphate phosphohydrolase 3-alpha",
  "term_label": "diadenosine pentaphosphate catabolic process",
  "gene": "UniProtKB:Q8NFP7",
  "gene_symbol": "NUDT10"
}